{
  "gene_name": "Serine_threonine-protein phosphatase 2A 56 kDa regulatory subunit delta isoform",
  "gene": "UniProtKB:Q14738",
  "term_id": "GO:0051177",
  "gene_symbol": "PPP2R5D",
  "term_label": "meiotic sister chromatid cohesion"
}